{
  "gene": "UniProtKB:Q06418",
  "term_id": "GO:0004714",
  "gene_name": "Tyrosine-protein kinase receptor TYRO3",
  "term_label": "transmembrane receptor protein tyrosine kinase activity",
  "gene_symbol": "TYRO3"
}